{
  "gene_name": "Histone H2B type 1-M",
  "gene": "UniProtKB:Q99879",
  "term_label": "structural constituent of chromatin",
  "term_id": "GO:0030527",
  "gene_symbol": "H2BC14"
}